{
  "term_id": "GO:0045597",
  "gene_name": "CCN family member 3",
  "term_label": "positive regulation of cell differentiation",
  "gene": "UniProtKB:P48745",
  "gene_symbol": "CCN3"
}